neuron differentiation involved in amphid sensory organ development [GO:0003387] (biological process) Sources: GOC:ascb_2009, GOC:dph, GOC:tb Relationships: is a type of GO:0030182; BFO_0000050 amphid sensory organ development [GO:0003386] Definition: The process in which a relatively unspecialized cell acquires specialized features of a neuron that contributes to the progression of the amphid sensory gland.